{
  "term_id": "UNKNOWN:0003",
  "gene": "UniProtKB:Q6GMV3",
  "gene_name": "Putative peptidyl-tRNA hydrolase PTRHD1",
  "term_label": "Unknown cellular component",
  "gene_symbol": "PTRHD1"
}